{
  "term_label": "cell adhesion mediated by integrin",
  "gene_symbol": "ITGB5",
  "gene": "UniProtKB:P18084",
  "term_id": "GO:0033627",
  "gene_name": "Integrin beta-5"
}